cell chemotaxis to angiotensin [GO:0071434] (biological process) Definition: The directed movement of a motile cell in response to the presence of angiotensin. Relationships: is a type of cell chemotaxis [GO:0060326] Also known as: angiotensin mediated chemotaxis, angiotensin-mediated cell chemotaxis Sources: GOC:mah